head morphogenesis [GO:0060323] (biological process) Sources: GOC:dph Definition: The process in which the anatomical structures of the head are generated and organized. The head is the anterior-most division of the body. Relationships: is a type of anatomical structure morphogenesis [GO:0009653]; is part of GO:0010171; is part of GO:0060322